{
  "gene": "UniProtKB:Q96NW4",
  "gene_name": "Ankyrin repeat domain-containing protein 27",
  "term_id": "GO:0043005",
  "term_label": "neuron projection",
  "gene_symbol": "ANKRD27"
}